{
  "gene_symbol": "LY6G6C",
  "gene": "UniProtKB:O95867",
  "term_id": "GO:0009897",
  "gene_name": "Lymphocyte antigen 6 complex locus protein G6c",
  "term_label": "external side of plasma membrane"
}